lithium ion export across the plasma membrane [GO:0010352] (biological process) References: PMID:17270011 Also known as: lithium export, lithium ion efflux, lithium ion export Definition: The directed movement of lithium ion out of a cell or organelle. Relationships: is a type of lithium ion transmembrane transport [GO:0090452]; is a type of export across plasma membrane [GO:0140115]